{
  "gene_name": "T cell receptor gamma variable 8",
  "gene": "UniProtKB:A0A0C4DH27",
  "term_label": "Unknown cellular component",
  "gene_symbol": "TRGV8",
  "term_id": "UNKNOWN:0003"
}